glycerate transmembrane transport [GO:1901975] (biological process) Relationships: is a type of GO:0034219; is a type of aldonate transmembrane transport [GO:0042873] References: PMID:23382251 Sources: GOC:TermGenie Definition: The process in which glycerate is transported across a membrane.